FACT complex assembly [GO:1905635] (biological process) Definition: The aggregation, arrangement and bonding together of a set of components to form a FACT complex. Relationships: is a type of protein-containing complex assembly [GO:0065003] Regulation: regulated by regulation of FACT complex assembly [GO:1905644]; negatively regulated by negative regulation of FACT complex assembly [GO:1905645]; positively regulated by positive regulation of FACT complex assembly [GO:1905646] References: PMID:20889714 Sources: GOC:TermGenie, GO_REF:0000079 Also known as: FACT complex formation, Facilitates chromatin transcription complex assembly, Facilitates chromatin transcription complex formation